DNA-binding transcription repressor activity [GO:0001217] (MF) Also known as: bacterial-type DNA binding transcription repressor activity, bacterial-type RNA polymerase core promoter proximal region sequence-specific DNA binding transcription factor activity involved in negative regulation of transcription, bacterial-type RNA polymerase transcriptional repressor activity, cadmium ion regulated sequence-specific DNA binding, bacterial-type RNA polymerase transcriptional repressor activity, copper ion regulated sequence-specific DNA binding, bacterial-type RNA polymerase transcriptional repressor activity, metal ion regulated sequence-specific DNA binding, bacterial-type RNA polymerase transcriptional repressor activity, sequence-specific DNA binding, cadmium ion regulated sequence-specific DNA binding bacterial-type RNA polymerase transcription factor activity involved in negative regulation of transcription, copper ion regulated sequence-specific DNA binding bacterial-type RNA polymerase transcription factor activity involved in negative regulation of transcription, metal ion regulated sequence-specific DNA binding bacterial-type RNA polymerase transcription factor activity involved in negative regulation of transcription, sequence-specific DNA binding bacterial-type RNA polymerase transcription factor activity involved in negative regulation of transcription, transcriptional repressor activity, bacterial-type RNA polymerase core promoter proximal region sequence-specific binding, transcriptional repressor activity, bacterial-type RNA polymerase proximal promoter sequence-specific DNA binding Subtypes: GO:0001227, DNA-binding transcription repressor activity, RNA polymerase III-specific [GO:0106250], GO:0141096 Sources: GOC:txnOH-2018 Note: For usage guidance, see comment in GO:0003700 ; DNA-binding transcription factor activity. Relationships: is a type of DNA-binding transcription factor activity [GO:0003700]; is part of negative regulation of DNA-templated transcription [GO:0045892] Definition: A DNA-binding transcription factor activity that represses or decreases the transcription of specific gene sets.